positive regulation of octopamine or tyramine signaling pathway [GO:2000127] (biological process) Relationships: is a type of GO:0045745; is a type of regulation of octopamine or tyramine signaling pathway [GO:2000125]; positively regulates octopamine or tyramine signaling pathway [GO:0007211] Also known as: positive regulation of octopamine or tyramine signalling pathway, positive regulation of octopamine/tyramine signaling pathway Sources: GOC:mah Definition: Any process that activates or increases the frequency, rate or extent of octopamine or tyramine signaling pathway. Subtypes: positive regulation of octopamine signaling pathway [GO:2000130], positive regulation of tyramine signaling pathway [GO:2000133]